presynaptic endocytic zone [GO:0098833] (cellular component) References: PMID:17455288 Relationships: is a type of cellular anatomical structure [GO:0110165]; is part of presynapse [GO:0098793] Definition: A specialized region of the plasma membrane and underlying cytoplasm which surround the the active zone, into which synaptic vesicle membranes are recycled following exocytosis. It is especially enriched in endocytic proteins following intense activity. Note: May be identical to periactive zone?